kidney stroma development [GO:0072072] (biological process) Definition: The process whose specific outcome is the progression of the kidney stroma over time, from its formation to the mature structure. The kidney stroma is the mesenchyme of the mature kidney. Sources: GOC:mtg_kidney_jan10 Relationships: is a type of connective tissue development [GO:0061448]; is a type of kidney mesenchyme development [GO:0072074]